{
  "term_id": "GO:0034472",
  "gene_name": "Integrator complex subunit 2",
  "gene": "UniProtKB:Q9H0H0",
  "gene_symbol": "INTS2",
  "term_label": "snRNA 3'-end processing"
}